{
  "gene_symbol": "CHCHD7",
  "term_id": "UNKNOWN:0001",
  "gene_name": "Coiled-coil-helix-coiled-coil-helix domain-containing protein 7",
  "term_label": "Unknown molecular function",
  "gene": "UniProtKB:Q9BUK0"
}